glutamate reuptake [GO:0051935] (biological process) Regulation: regulated by regulation of glutamate uptake involved in transmission of nerve impulse [GO:0051946]; negatively regulated by negative regulation of glutamate uptake involved in transmission of nerve impulse [GO:0051948]; positively regulated by GO:0051951 Sources: ISBN:0123668387, Wikipedia:Glutamate_transporter Definition: The uptake of L-glutamate by neurons or glial cells. This process leads to inactivation and recycling of neurotransmitters. Relationships: is a type of GO:0051933; is a type of L-glutamate import across plasma membrane [GO:0098712] Also known as: glutamate recycling, L-glutamate reuptake, L-glutamate uptake involved in synaptic transmission, glutamate import into glial cell, glutamate import into neuron, L-glutamate uptake during transmission of nerve impulse, glutamate uptake during transmission of nerve impulse